chemorepulsion of axon [GO:0061643] (biological process) Definition: The process in which a neuron growth cone is directed to a specific target site in response to a repulsive chemical cue. Relationships: is_a negative chemotaxis [GO:0050919]; is part of GO:0007411; is part of cellular response to chemical stimulus [GO:0070887] Sources: GOC:dph, GOC:krc Subtypes: chemorepulsion of branchiomotor axon [GO:0021793], chemorepulsion of dopaminergic neuron axon [GO:0036518], chemorepulsion of serotonergic neuron axon [GO:0036519]